{
  "term_label": "RNA polymerase II cis-regulatory region sequence-specific DNA binding",
  "gene_name": "Transcription factor YY2",
  "gene_symbol": "YY2",
  "gene": "UniProtKB:O15391",
  "term_id": "GO:0000978"
}